{
  "gene": "UniProtKB:Q9NSK0",
  "term_id": "GO:0007018",
  "gene_symbol": "KLC4",
  "gene_name": "Kinesin light chain 4",
  "term_label": "microtubule-based movement"
}